regulation of CD8-positive, alpha-beta cytotoxic T cell extravasation [GO:2000452] (biological process) Definition: Any process that modulates the frequency, rate or extent of CD8-positive, alpha-beta cytotoxic T cell extravasation. Subtypes: negative regulation of CD8-positive, alpha-beta cytotoxic T cell extravasation [GO:2000453], positive regulation of CD8-positive, alpha-beta cytotoxic T cell extravasation [GO:2000454] Sources: GOC:obol Relationships: is a type of regulation of CD8-positive, alpha-beta T cell extravasation [GO:2000449]; regulates CD8-positive, alpha-beta cytotoxic T cell extravasation [GO:0035698]